{
  "gene_name": "Protein Wnt-11",
  "term_id": "GO:0005125",
  "gene": "UniProtKB:O96014",
  "gene_symbol": "WNT11",
  "term_label": "cytokine activity"
}